{
  "gene": "UniProtKB:Q8NHW3",
  "gene_name": "Transcription factor MafA",
  "gene_symbol": "MAFA",
  "term_label": "response to glucose",
  "term_id": "GO:0009749"
}